detection of high humidity stimulus involved in sensory perception [GO:0098514] (biological process) References: PMID:18269908 Sources: GOC:dos Definition: The series of events in which a high humidity stimulus is detected and converted into a molecular signal as a part of the sensory detection of high humidity. Relationships: is a type of detection of humidity stimulus involved in sensory perception [GO:0098512]; is a type of detection of high humidity [GO:0098516]; is part of sensory perception of high humidity [GO:0098510]